{
  "gene": "UniProtKB:O14791",
  "gene_name": "Apolipoprotein L1",
  "term_label": "Unknown cellular component",
  "term_id": "UNKNOWN:0003",
  "gene_symbol": "APOL1"
}